{
  "gene": "UniProtKB:Q8TAM2",
  "gene_symbol": "TTC8",
  "gene_name": "Tetratricopeptide repeat protein 8",
  "term_label": "Unknown molecular function",
  "term_id": "UNKNOWN:0001"
}